{
  "gene": "UniProtKB:O14950",
  "gene_symbol": "MYL12B",
  "gene_name": "Myosin regulatory light chain 12B",
  "term_label": "stress fiber",
  "term_id": "GO:0001725"
}